nucleotide-sulfate transport [GO:0015715] (BP) Definition: The directed movement of nucleotide sulfate into, out of or within a cell, or between cells, by means of some agent such as a transporter or pore. Relationships: is a type of organophosphate ester transport [GO:0015748]; is a type of GO:0015931; is_a GO:0072348 Sources: GOC:mah Also known as: nucleotide-sulphate transport